{
  "term_label": "DNA binding",
  "term_id": "GO:0003677",
  "gene_symbol": "RLF",
  "gene_name": "Zinc finger protein Rlf",
  "gene": "UniProtKB:Q13129"
}